{
  "gene_name": "PX domain-containing protein 1",
  "term_label": "Unknown molecular function",
  "gene_symbol": "PXDC1",
  "term_id": "UNKNOWN:0001",
  "gene": "UniProtKB:Q5TGL8"
}